{
  "gene": "UniProtKB:P14651",
  "term_label": "regulation of transcription by RNA polymerase II",
  "gene_symbol": "HOXB3",
  "gene_name": "Homeobox protein Hox-B3",
  "term_id": "GO:0006357"
}